beta-glucuronidase activity [GO:0004566] (molecular function) Definition: Catalysis of the reaction: a beta-D-glucuronoside + H2O = an alcohol + D-glucuronate. Relationships: is a type of glucuronidase activity [GO:0046574] Also known as: beta-D-glucuronoside glucuronosohydrolase activity, beta-glucuronide glucuronohydrolase activity, exo-beta-D-glucuronidase activity, glucuronidase activity, ketodase activity Sources: EC:3.2.1.31